1-phosphofructokinase activity [GO:0008662] (molecular function) Definition: Catalysis of the reaction: ATP + D-fructose 1-phosphate = ADP + D-fructose 1,6-bisphosphate. Sources: EC:2.7.1.56 Also known as: 1-phosphofructokinase (phosphorylating), ATP:D-fructose-phosphate 6-phosphotransferase activity, D-fructose-1-phosphate kinase activity, fructose 1-phosphate kinase activity, fructose-1-phosphate kinase activity, phosphofructokinase 1 Relationships: is a type of phosphofructokinase activity [GO:0008443]